{
  "gene": "UniProtKB:A6NNV3",
  "gene_symbol": "SPDYE16",
  "gene_name": "Putative speedy protein E16",
  "term_label": "Unknown cellular component",
  "term_id": "UNKNOWN:0003"
}